{
  "gene_name": "THAP domain-containing protein 7",
  "gene_symbol": "THAP7",
  "term_id": "UNKNOWN:0001",
  "gene": "UniProtKB:Q9BT49",
  "term_label": "Unknown molecular function"
}